positive regulation of CAMKK-AMPK signaling cascade [GO:1905291] (biological process) Definition: Any process that activates or increases the frequency, rate or extent of CAMKK-AMPK signaling cascade. References: PMID:22128786 Sources: GOC:TermGenie, GO_REF:0000058 Also known as: up regulation of CAMKK-AMPK signaling cascade, up-regulation of CAMKK-AMPK signaling cascade, upregulation of CAMKK-AMPK signaling cascade, activation of CAMKK-AMPK signaling cascade, activation of stress-activated AMP-activated protein kinase signaling cascade, positive regulation of stress-activated AMP-activated protein kinase signaling cascade, up regulation of stress-activated AMP-activated protein kinase signaling cascade, up-regulation of stress-activated AMP-activated protein kinase signaling cascade, upregulation of stress-activated AMP-activated protein kinase signaling cascade Relationships: is a type of positive regulation of calcium-mediated signaling [GO:0050850]; is a type of regulation of CAMKK-AMPK signaling cascade [GO:1905289]; positively regulates CAMKK-AMPK signaling cascade [GO:0061762]